{
  "gene": "UniProtKB:Q70EL1",
  "term_label": "Unknown biological process",
  "term_id": "UNKNOWN:0002",
  "gene_symbol": "USP54",
  "gene_name": "Inactive ubiquitin carboxyl-terminal hydrolase 54"
}